{
  "gene": "UniProtKB:Q6NUS8",
  "gene_name": "UDP-glucuronosyltransferase 3A1",
  "term_label": "glucuronosyltransferase activity",
  "gene_symbol": "UGT3A1",
  "term_id": "GO:0015020"
}